{
  "gene_name": "PRKCA-binding protein",
  "term_id": "GO:0006886",
  "gene_symbol": "PICK1",
  "term_label": "intracellular protein transport",
  "gene": "UniProtKB:Q9NRD5"
}